{
  "term_label": "extracellular space",
  "gene": "UniProtKB:P51888",
  "gene_name": "Prolargin",
  "term_id": "GO:0005615",
  "gene_symbol": "PRELP"
}